{
  "gene_name": "Protein PET117 homolog, mitochondrial",
  "term_label": "Unknown molecular function",
  "gene": "UniProtKB:Q6UWS5",
  "gene_symbol": "PET117",
  "term_id": "UNKNOWN:0001"
}